{
  "term_id": "GO:0052658",
  "gene_name": "Synaptojanin-1",
  "term_label": "inositol-1,4,5-trisphosphate 5-phosphatase activity",
  "gene": "UniProtKB:O43426",
  "gene_symbol": "SYNJ1"
}